{
  "term_label": "cytoplasm",
  "gene": "UniProtKB:P29377",
  "gene_name": "Protein S100-G",
  "gene_symbol": "S100G",
  "term_id": "GO:0005737"
}